{
  "gene": "UniProtKB:Q13868",
  "gene_name": "Exosome complex component RRP4",
  "term_label": "nuclear polyadenylation-dependent rRNA catabolic process",
  "term_id": "GO:0071035",
  "gene_symbol": "EXOSC2"
}